{
  "term_id": "GO:0030856",
  "gene_name": "Trans-acting T-cell-specific transcription factor GATA-3",
  "term_label": "regulation of epithelial cell differentiation",
  "gene_symbol": "GATA3",
  "gene": "UniProtKB:P23771"
}